regulation of ferrichrome biosynthetic process [GO:1905568] (biological process) Also known as: regulation of ferrichrome anabolism, regulation of ferrichrome biosynthesis, regulation of ferrichrome formation, regulation of ferrichrome synthesis, regulation of ferrichrome biosynthetic process, peptide formation, regulation of ferrichrome biosynthetic process, peptide modification Definition: Any process that modulates the frequency, rate or extent of ferrichrome biosynthetic process. Relationships: is a type of regulation of amide metabolic process [GO:0034248]; is a type of regulation of siderophore biosynthetic process [GO:1900704]; regulates ferrichrome biosynthetic process [GO:0031169] Subtypes: regulation of ferricrocin biosynthetic process [GO:1900678], negative regulation of ferrichrome biosynthetic process [GO:1905569], positive regulation of ferrichrome biosynthetic process [GO:1905570] Sources: GOC:TermGenie, GOC:al, GO_REF:0000058